{
  "term_id": "GO:0031902",
  "term_label": "late endosome membrane",
  "gene": "UniProtKB:Q9UEU0",
  "gene_name": "Vesicle transport through interaction with t-SNAREs homolog 1B",
  "gene_symbol": "VTI1B"
}